negative regulation of odontogenesis of dentin-containing tooth [GO:0042489] (biological process) Also known as: down regulation of odontogenesis, down-regulation of odontogenesis, downregulation of odontogenesis, inhibition of odontogenesis, negative regulation of odontogenesis, negative regulation of odontogenesis of dentine-containing teeth, negative regulation of odontogenesis of dentine-containing tooth Definition: Any process that stops, prevents, or reduces the frequency, rate or extent of the formation and development of teeth, the hard, bony appendages which are borne on the jaws, or on other bones in the walls of the mouth or pharynx. Relationships: is a type of negative regulation of odontogenesis [GO:0042483]; is a type of regulation of odontogenesis of dentin-containing tooth [GO:0042487]; RO_0002212 odontogenesis of dentin-containing tooth [GO:0042475] References: PMID:15355794 Sources: GOC:jl, GOC:mtg_sensu